{
  "gene_symbol": "ANKRD60",
  "gene": "UniProtKB:Q9BZ19",
  "term_id": "UNKNOWN:0001",
  "term_label": "Unknown molecular function",
  "gene_name": "Ankyrin repeat domain-containing protein 60"
}